6-carboxytetrahydropterin synthase activity [GO:0070497] (molecular function) Definition: Catalysis of the reaction: 7,8-dihydroneopterin triphosphate + H2O = 6-carboxy-5,6,7,8-tetrahydropterin + triphosphate + acetaldehyde + 2 H+. Also known as: 6-carboxy-5,6,7,8-tetrahydropterin synthase activity References: PMID:19231875 Sources: GOC:imk, RHEA:27966 Relationships: is a type of hydro-lyase activity [GO:0016836]